{
  "gene_symbol": "ASCL3",
  "gene": "UniProtKB:Q9NQ33",
  "gene_name": "Achaete-scute homolog 3",
  "term_id": "GO:0000981",
  "term_label": "DNA-binding transcription factor activity, RNA polymerase II-specific"
}